{
  "term_id": "GO:0010592",
  "term_label": "positive regulation of lamellipodium assembly",
  "gene_symbol": "RAC2",
  "gene_name": "Ras-related C3 botulinum toxin substrate 2",
  "gene": "UniProtKB:P15153"
}